{
  "gene": "UniProtKB:Q9Y232",
  "term_id": "GO:0003714",
  "gene_name": "Chromodomain Y-like protein",
  "gene_symbol": "CDYL",
  "term_label": "transcription corepressor activity"
}